{
  "term_label": "extracellular space",
  "gene": "UniProtKB:P07942",
  "term_id": "GO:0005615",
  "gene_symbol": "LAMB1",
  "gene_name": "Laminin subunit beta-1"
}